{
  "term_label": "innate immune response",
  "gene_name": "Tripartite motif-containing protein 55",
  "term_id": "GO:0045087",
  "gene": "UniProtKB:Q9BYV6",
  "gene_symbol": "TRIM55"
}